{
  "term_id": "UNKNOWN:0002",
  "term_label": "Unknown biological process",
  "gene_name": "Transmembrane protein 192",
  "gene": "UniProtKB:Q8IY95",
  "gene_symbol": "TMEM192"
}